{
  "gene_symbol": "TMPRSS11A",
  "term_id": "GO:0008236",
  "term_label": "serine-type peptidase activity",
  "gene": "UniProtKB:Q6ZMR5",
  "gene_name": "Transmembrane protease serine 11A"
}